{
  "term_label": "CXCR chemokine receptor binding",
  "gene_symbol": "CXCL6",
  "gene_name": "C-X-C motif chemokine 6",
  "gene": "UniProtKB:P80162",
  "term_id": "GO:0045236"
}